{
  "gene": "UniProtKB:P01036",
  "gene_symbol": "CST4",
  "term_id": "UNKNOWN:0002",
  "gene_name": "Cystatin-S",
  "term_label": "Unknown biological process"
}